positive regulation of toll-like receptor 6 signaling pathway [GO:0034153] (biological process) Definition: Any process that activates or increases the frequency, rate, or extent of toll-like receptor 6 signaling pathway. References: PMID:16551253, PMID:17328678 Sources: GOC:add Also known as: positive regulation of TLR6 signaling pathway, positive regulation of toll-like receptor 6 signalling pathway Relationships: is a type of GO:0034151; is a type of GO:0062208; positively regulates GO:0034150